{
  "term_id": "GO:0045921",
  "gene": "UniProtKB:Q86UW7",
  "gene_symbol": "CADPS2",
  "term_label": "positive regulation of exocytosis",
  "gene_name": "Calcium-dependent secretion activator 2"
}